{
  "term_id": "GO:0046332",
  "gene_symbol": "SKI",
  "term_label": "SMAD binding",
  "gene": "UniProtKB:P12755",
  "gene_name": "Ski oncogene"
}